mitochondrial tryptophanyl-tRNA aminoacylation [GO:0070183] (biological process) Sources: GOC:mah, GOC:mcc Definition: The process of coupling tryptophan to tryptophanyl-tRNA in a mitochondrion, catalyzed by tryptophanyl-tRNA synthetase. In tRNA aminoacylation, the amino acid is first activated by linkage to AMP and then transferred to either the 2'- or the 3'-hydroxyl group of the 3'-adenosine residue of the tRNA. Relationships: is a type of tryptophanyl-tRNA aminoacylation [GO:0006436]; is a type of GO:0070127